{
  "gene_symbol": "C1orf226",
  "gene": "UniProtKB:A1L170",
  "gene_name": "Uncharacterized protein C1orf226",
  "term_id": "UNKNOWN:0003",
  "term_label": "Unknown cellular component"
}